{
  "gene_name": "Heparan sulfate glucosamine 3-O-sulfotransferase 5",
  "term_label": "Unknown cellular component",
  "gene": "UniProtKB:Q8IZT8",
  "gene_symbol": "HS3ST5",
  "term_id": "UNKNOWN:0003"
}